positive regulation of natural killer cell mediated immune response to tumor cell [GO:0002857] (biological process) Also known as: up regulation of natural killer cell mediated immune response to tumor cell, up-regulation of natural killer cell mediated immune response to tumor cell, upregulation of natural killer cell mediated immune response to tumor cell, activation of natural killer cell mediated immune response to tumor cell, stimulation of natural killer cell mediated immune response to tumor cell Subtypes: GO:0002860 Definition: Any process that activates or increases the frequency, rate, or extent of natural killer cell mediated immune response to a tumor cell. Relationships: is a type of positive regulation of natural killer cell mediated immunity [GO:0002717]; is a type of positive regulation of immune response to tumor cell [GO:0002839]; is a type of regulation of natural killer cell mediated immune response to tumor cell [GO:0002855]; positively regulates natural killer cell mediated immune response to tumor cell [GO:0002423] Sources: GOC:add